kidney cortex tubule cell dedifferentiation [GO:0160029] (BP) Relationships: is a type of cell dedifferentiation [GO:0043697] References: PMID:18987110, PMID:31847447 Note: Following injury, renal cortex tubular epithelial cell appears to be undergoing epithelial-mesenchymal transition, detected by overexpression of vimentin. Definition: The process in which a kidney cortex tubule cell (specialized epithelial cell of the kidney) loses the structural or functional features that characterize it in the mature organism, or some other relatively stable phase of the organism's life history. Under certain conditions, these cells can revert back to the features of the stem cells that were their ancestors.